{
  "gene": "UniProtKB:Q4KMQ1",
  "term_id": "GO:0060088",
  "term_label": "auditory receptor cell stereocilium organization",
  "gene_symbol": "TPRN",
  "gene_name": "Taperin"
}